{
  "gene_symbol": "LOC122513141",
  "gene_name": "RING-type domain-containing protein",
  "gene": "UniProtKB:A0A2R8Y4M4",
  "term_label": "endoplasmic reticulum membrane",
  "term_id": "GO:0005789"
}